tricuspid valve development [GO:0003175] (biological process) Definition: The progression of the tricuspid valve over time, from its formation to the mature structure. Sources: GOC:mtg_heart Relationships: is a type of atrioventricular valve development [GO:0003171]